{
  "gene_symbol": "NCBP1",
  "term_label": "nucleus",
  "gene": "UniProtKB:Q09161",
  "term_id": "GO:0005634",
  "gene_name": "Nuclear cap-binding protein subunit 1"
}